oncostatin-M receptor complex [GO:0005900] (cellular component) References: PMID:8999038 Sources: GOC:jl Relationships: is a type of GO:0098802 Definition: A heterodimeric receptor for the cytokine oncostatin-M (OSM). In humans the receptor complex is made up of the gene products gp130 and OSMR-beta.